{
  "term_id": "GO:0030048",
  "gene_name": "Unconventional myosin-Ic",
  "term_label": "actin filament-based movement",
  "gene": "UniProtKB:O00159",
  "gene_symbol": "MYO1C"
}